regulation of dauer larval development [GO:0061065] (biological process) Subtypes: GO:0061066, GO:0061067, regulation of dauer entry [GO:1905909] Definition: Any process that modulates the rate, frequency, or extent of dauer larval development, the process whose specific outcome is the progression of the dauer larva over time, through the facultative diapause of the dauer (enduring) larval stage, with specialized traits adapted for dispersal and long-term survival, with elevated stress resistance and without feeding. Relationships: is a type of regulation of nematode larval development [GO:0061062]; regulates dauer larval development [GO:0040024] Sources: GOC:dph, GOC:kmv